{
  "term_id": "GO:0030154",
  "gene_name": "Forkhead box protein C1",
  "gene_symbol": "FOXC1",
  "gene": "UniProtKB:Q12948",
  "term_label": "cell differentiation"
}